UDP biosynthetic process [GO:0006225] (biological process) Definition: The chemical reactions and pathways resulting in the formation of UDP, uridine (5'-)diphosphate. Also known as: UDP anabolism, UDP biosynthesis, UDP formation, UDP synthesis Relationships: is a type of GO:0009194; is_a pyrimidine ribonucleotide biosynthetic process [GO:0009220]; is a type of GO:0046048 Sources: ISBN:0198506732